histone H1 methyltransferase activity [GO:0140188] (molecular function) Also known as: histone H1 methylase activity, histone H1 methylation Definition: Catalysis of the reaction: S-adenosyl-L-methionine + a histone H1 = S-adenosyl-L-homocysteine + a methylated histone H1. References: PMID:19144645 Subtypes: H1-4K26 methyltransferase activity [GO:0140189] Relationships: is a type of histone methyltransferase activity [GO:0042054]